{
  "term_label": "Unknown biological process",
  "term_id": "UNKNOWN:0002",
  "gene_symbol": "ARRDC1-AS1",
  "gene_name": "Uncharacterized protein ARRDC1-AS1",
  "gene": "UniProtKB:Q9H2J1"
}